cellular response to ionizing radiation [GO:0071479] (biological process) Sources: GOC:mah Also known as: cellular response to ionising radiation, cellular response to ionizing radiation stimulus Definition: Any process that results in a change in state or activity of a cell (in terms of movement, secretion, enzyme production, gene expression, etc.) as a result of a ionizing radiation stimulus. Ionizing radiation is radiation with sufficient energy to remove electrons from atoms and may arise from spontaneous decay of unstable isotopes, resulting in alpha and beta particles and gamma rays. Ionizing radiation also includes X-rays. Relationships: is a type of response to ionizing radiation [GO:0010212]; is_a cellular response to radiation [GO:0071478] Subtypes: cellular response to gamma radiation [GO:0071480], cellular response to X-ray [GO:0071481]